positive regulation of colon smooth muscle contraction [GO:1904343] (biological process) References: PMID:24170253 Sources: GOC:TermGenie, GO_REF:0000058 Also known as: up regulation of colon smooth muscle contraction, up-regulation of colon smooth muscle contraction, upregulation of colon smooth muscle contraction, activation of colon smooth muscle contraction Definition: Any process that activates or increases the frequency, rate or extent of colon smooth muscle contraction. Relationships: is a type of positive regulation of gastro-intestinal system smooth muscle contraction [GO:1904306]; is a type of GO:1904341; positively regulates colon smooth muscle contraction [GO:1990765]